{
  "gene_symbol": "TNFAIP6",
  "gene_name": "Tumor necrosis factor-inducible gene 6 protein",
  "gene": "UniProtKB:P98066",
  "term_id": "GO:0005615",
  "term_label": "extracellular space"
}